{
  "term_label": "poly-N-acetyllactosamine biosynthetic process",
  "term_id": "GO:0030311",
  "gene": "UniProtKB:Q7Z7M8",
  "gene_symbol": "B3GNT8",
  "gene_name": "UDP-GlcNAc:betaGal beta-1,3-N-acetylglucosaminyltransferase 8"
}